{
  "gene": "UniProtKB:Q96RT1",
  "gene_symbol": "ERBIN",
  "term_label": "Unknown molecular function",
  "gene_name": "Erbin",
  "term_id": "UNKNOWN:0001"
}